{
  "gene_name": "Tyrosyl-DNA phosphodiesterase 2",
  "gene": "UniProtKB:O95551",
  "term_label": "double-strand break repair",
  "term_id": "GO:0006302",
  "gene_symbol": "TDP2"
}